{
  "gene": "UniProtKB:Q15911",
  "term_id": "GO:0006357",
  "gene_name": "Zinc finger homeobox protein 3",
  "gene_symbol": "ZFHX3",
  "term_label": "regulation of transcription by RNA polymerase II"
}